{
  "gene_symbol": "PADI2",
  "gene_name": "Protein-arginine deiminase type-2",
  "gene": "UniProtKB:Q9Y2J8",
  "term_id": "GO:0005737",
  "term_label": "cytoplasm"
}